{
  "gene_name": "Coiled-coil domain-containing protein 63",
  "gene_symbol": "CCDC63",
  "term_label": "axoneme",
  "term_id": "GO:0005930",
  "gene": "UniProtKB:Q8NA47"
}